{
  "gene": "UniProtKB:Q9UMR2",
  "term_id": "GO:0016973",
  "gene_symbol": "DDX19B",
  "gene_name": "ATP-dependent RNA helicase DDX19B",
  "term_label": "poly(A)+ mRNA export from nucleus"
}